taxis to electron acceptor [GO:0042334] (biological process) Also known as: taxis in response to electron acceptor References: PMID:11029423 Sources: GOC:jl Definition: The directed movement of a motile cell or organism in response to the presence of an alternative electron acceptor, for example, nitrate. Relationships: is a type of energy taxis [GO:0009453]